{
  "gene_symbol": "ZW10",
  "gene": "UniProtKB:O43264",
  "gene_name": "Centromere_kinetochore protein zw10 homolog",
  "term_id": "UNKNOWN:0001",
  "term_label": "Unknown molecular function"
}